{
  "term_id": "UNKNOWN:0003",
  "gene_symbol": "OR5AC1",
  "gene": "UniProtKB:P0C628",
  "term_label": "Unknown cellular component",
  "gene_name": "Olfactory receptor 5AC1"
}